{
  "term_id": "GO:0004439",
  "term_label": "phosphatidylinositol-4,5-bisphosphate 5-phosphatase activity",
  "gene": "UniProtKB:Q15735",
  "gene_name": "Phosphatidylinositol 4,5-bisphosphate 5-phosphatase A",
  "gene_symbol": "INPP5J"
}